{
  "gene_name": "Gamma-aminobutyric acid receptor subunit alpha-4",
  "gene_symbol": "GABRA4",
  "gene": "UniProtKB:P48169",
  "term_label": "chloride transmembrane transport",
  "term_id": "GO:1902476"
}